{
  "gene_symbol": "OR52N4",
  "gene_name": "Olfactory receptor 52N4",
  "term_id": "GO:0004984",
  "term_label": "olfactory receptor activity",
  "gene": "UniProtKB:Q8NGI2"
}